{
  "term_label": "cytoplasm",
  "gene_symbol": "BIRC5",
  "gene": "UniProtKB:O15392",
  "gene_name": "Baculoviral IAP repeat-containing protein 5",
  "term_id": "GO:0005737"
}